{
  "term_label": "(2E,6E)-farnesyl diphosphate synthase activity",
  "gene_name": "Farnesyl pyrophosphate synthase",
  "term_id": "GO:0004337",
  "gene_symbol": "FDPS",
  "gene": "UniProtKB:P14324"
}